{
  "term_label": "sarcolemma",
  "gene_name": "Delta-sarcoglycan",
  "gene_symbol": "SGCD",
  "term_id": "GO:0042383",
  "gene": "UniProtKB:Q92629"
}